{
  "gene": "UniProtKB:Q96NT5",
  "gene_name": "Proton-coupled folate transporter",
  "gene_symbol": "SLC46A1",
  "term_id": "GO:0005886",
  "term_label": "plasma membrane"
}